{
  "gene_symbol": "TRAV9-1",
  "gene": "UniProtKB:A0A075B6T8",
  "gene_name": "T cell receptor alpha variable 9-1",
  "term_id": "GO:0002250",
  "term_label": "adaptive immune response"
}